{
  "gene_symbol": "HSPA7",
  "term_label": "ATP hydrolysis activity",
  "gene_name": "Putative heat shock 70 kDa protein 7",
  "term_id": "GO:0016887",
  "gene": "UniProtKB:P48741"
}